{
  "term_id": "GO:0004435",
  "gene_symbol": "PLCB1",
  "term_label": "phosphatidylinositol-4,5-bisphosphate phospholipase C activity",
  "gene": "UniProtKB:Q9NQ66",
  "gene_name": "1-phosphatidylinositol 4,5-bisphosphate phosphodiesterase beta-1"
}